positive regulation of collateral sprouting of injured axon [GO:0048694] (biological process) Also known as: up regulation of collateral sprouting of injured axon, up-regulation of collateral sprouting of injured axon, upregulation of collateral sprouting of injured axon, activation of collateral sprouting of injured axon, stimulation of collateral sprouting of injured axon Definition: Any process that activates, maintains or increases the rate of collateral sprouting of an injured axon. Relationships: is a type of positive regulation of collateral sprouting [GO:0048672]; is a type of GO:0048687; is a type of GO:0048693; positively regulates collateral sprouting of injured axon [GO:0048674] Sources: GOC:dgh, GOC:dph, GOC:jid, GOC:lm